{
  "term_label": "L-amino acid transmembrane transporter activity",
  "gene": "UniProtKB:Q9UHI5",
  "term_id": "GO:0015179",
  "gene_name": "Large neutral amino acids transporter small subunit 2",
  "gene_symbol": "SLC7A8"
}